{
  "term_label": "Unknown cellular component",
  "gene": "UniProtKB:Q5TF39",
  "gene_name": "Sodium-dependent glucose transporter 1",
  "term_id": "UNKNOWN:0003",
  "gene_symbol": "MFSD4B"
}